{
  "gene_symbol": "G6PC1",
  "term_id": "GO:0016020",
  "gene": "UniProtKB:P35575",
  "term_label": "membrane",
  "gene_name": "Glucose-6-phosphatase catalytic subunit 1"
}